{
  "term_id": "UNKNOWN:0001",
  "gene_name": "MAP3K7 C-terminal-like protein",
  "term_label": "Unknown molecular function",
  "gene_symbol": "MAP3K7CL",
  "gene": "UniProtKB:P57077"
}